{
  "gene_name": "Neuroblastoma breakpoint family member 20",
  "gene_symbol": "NBPF20",
  "gene": "UniProtKB:P0DPF2",
  "term_label": "Unknown molecular function",
  "term_id": "UNKNOWN:0001"
}